{
  "gene": "UniProtKB:Q8TAV4",
  "gene_symbol": "STOML3",
  "term_label": "Unknown biological process",
  "gene_name": "Stomatin-like protein 3",
  "term_id": "UNKNOWN:0002"
}